regulation of dauer entry [GO:1905909] (BP) References: PMID:21531333 Sources: GOC:TermGenie, GO_REF:0000058 Definition: Any process that modulates the frequency, rate or extent of dauer entry. Relationships: is a type of regulation of dauer larval development [GO:0061065]; regulates dauer entry [GO:0043053] Also known as: regulation of nematode entry into dormancy Subtypes: negative regulation of dauer entry [GO:1905910], GO:1905911